{
  "term_label": "corticotropin hormone receptor binding",
  "gene_symbol": "MRAP2",
  "gene_name": "Melanocortin-2 receptor accessory protein 2",
  "term_id": "GO:0031780",
  "gene": "UniProtKB:Q96G30"
}